{
  "gene": "UniProtKB:O43615",
  "term_id": "GO:0030150",
  "gene_symbol": "TIMM44",
  "term_label": "protein import into mitochondrial matrix",
  "gene_name": "Mitochondrial import inner membrane translocase subunit TIM44"
}